{
  "term_id": "GO:0006693",
  "gene": "UniProtKB:Q14914",
  "term_label": "prostaglandin metabolic process",
  "gene_name": "Prostaglandin reductase 1",
  "gene_symbol": "PTGR1"
}